taurine:sodium symporter activity [GO:0005369] (molecular function) Relationships: is a type of organic acid:sodium symporter activity [GO:0005343]; is a type of taurine transmembrane transporter activity [GO:0005368] Definition: Enables the transfer of a solute or solutes from one side of a membrane to the other according to the reaction: taurine(out) + Na+(out) = taurine(in) + Na+(in). Also known as: sodium/chloride-dependent taurine transporter Sources: TC:2.A.22.3.3